{
  "gene_name": "E3 ubiquitin ligase TRAF3IP2",
  "gene": "UniProtKB:O43734",
  "gene_symbol": "TRAF3IP2",
  "term_label": "positive regulation of canonical NF-kappaB signal transduction",
  "term_id": "GO:0043123"
}